histone H4 reader activity [GO:0140008] (molecular function) Subtypes: histone H4K20me2 reader activity [GO:0140005], GO:0140011, histone H4K5ac reader activity [GO:0140012], histone H4K16ac reader activity [GO:0140046], GO:0140055, histone H4K20me1 reader activity [GO:0140117], histone H4K20me3 reader activity [GO:1990889] Definition: A histone reader that specifically binds either to an unmodified histone H4 or a form modified by a post-translational modification on a specific residue. The most common PTMs on histones are methylation, acetylation and phosphorylation. Relationships: is a type of histone reader activity [GO:0140566] References: PMID:11498575, PMID:25688442, PMID:31082667, PMID:34726351